{
  "gene_name": "Protein salvador homolog 1",
  "term_id": "GO:0035329",
  "gene": "UniProtKB:Q9H4B6",
  "term_label": "hippo signaling",
  "gene_symbol": "SAV1"
}